{
  "gene_name": "Cytochrome b",
  "term_id": "GO:0016020",
  "term_label": "membrane",
  "gene": "UniProtKB:P00156",
  "gene_symbol": "MT-CYB"
}